{
  "term_id": "GO:0032422",
  "term_label": "purine-rich negative regulatory element binding",
  "gene": "UniProtKB:Q9UJV8",
  "gene_name": "Purine-rich element-binding protein gamma",
  "gene_symbol": "PURG"
}